visual perception [GO:0007601] (biological process) Sources: GOC:ai Definition: The series of events required for an organism to receive a visual stimulus, convert it to a molecular signal, and recognize and characterize the signal. Visual stimuli are detected in the form of photons and are processed to form an image. Relationships: is a type of sensory perception of light stimulus [GO:0050953] Also known as: sense of sight, sensory visual perception, vision Subtypes: visual perception involved in equilibrioception [GO:0051356]